{
  "gene_name": "Thrombospondin type-1 domain-containing protein 8",
  "gene_symbol": "THSD8",
  "gene": "UniProtKB:A0A1W2PP97",
  "term_label": "Unknown cellular component",
  "term_id": "UNKNOWN:0003"
}